{
  "gene_symbol": "SCIMP",
  "term_label": "Unknown molecular function",
  "gene": "UniProtKB:Q6UWF3",
  "term_id": "UNKNOWN:0001",
  "gene_name": "SLP adapter and CSK-interacting membrane protein"
}